{
  "term_id": "GO:0000978",
  "gene_name": "Homeobox protein DLX-1",
  "gene_symbol": "DLX1",
  "term_label": "RNA polymerase II cis-regulatory region sequence-specific DNA binding",
  "gene": "UniProtKB:P56177"
}